smooth endoplasmic reticulum cisterna [GO:0120082] (cellular component) References: PMID:12112448 Sources: GOC:sl Definition: A subcompartment of the smooth endoplasmic reticulum consisting of lumenal expansion into a flattened, disc-shaped cavity. Subtypes: subrhabdomeral cisterna [GO:0016029], GO:1990039 Relationships: is a type of GO:0110165; is part of smooth endoplasmic reticulum [GO:0005790]; is part of endoplasmic reticulum cisternal network [GO:0071781]